{
  "gene": "UniProtKB:Q9H5P4",
  "term_label": "Unknown molecular function",
  "term_id": "UNKNOWN:0001",
  "gene_symbol": "PDZD7",
  "gene_name": "PDZ domain-containing protein 7"
}